endonucleolytic cleaveage between LSU-rRNA and 4.5S rRNA of tetracistronic rRNA transcript (SSU-rRNA, LSU-rRNA, 4.5S-rRNA, 5S-rRNA) [GO:0002105] (biological process) Definition: Endonucleolytic cleavage between the LSU-rRNA and the 4.5S rRNA of an rRNA molecule originally produced as a tetracistronic rRNA transcript that contains the Small Subunit (SSU) rRNA, Large Subunit (LSU) the 4.5S rRNA, and the 5S rRNA in that order from 5' to 3' along the primary transcript. Note that the use of the word tetracistronic refers only to the number of mature rRNA molecules which will be produced from the primary transcript and ignores tRNAs that may also be present within the primary transcript. Relationships: is a type of GO:0002103 Sources: GOC:curators